{
  "gene": "UniProtKB:P10720",
  "term_label": "antimicrobial humoral immune response mediated by antimicrobial peptide",
  "term_id": "GO:0061844",
  "gene_symbol": "PF4V1",
  "gene_name": "Platelet factor 4 variant"
}